transepithelial ammonium transport [GO:0070634] (biological process) Definition: The directed movement of ammonium ions from one side of an epithelium to the other. Relationships: is a type of transepithelial transport [GO:0070633]; is a type of nitrogen compound transport [GO:0071705] Sources: GOC:mah, GOC:yaf